{
  "term_id": "GO:0006622",
  "gene": "UniProtKB:P20645",
  "gene_symbol": "M6PR",
  "gene_name": "Cation-dependent mannose-6-phosphate receptor",
  "term_label": "protein targeting to lysosome"
}